negative regulation of gut granule assembly [GO:1904756] (biological process) References: PMID:17535251 Sources: GOC:TermGenie, GO_REF:0000058 Also known as: down regulation of gut granule assembly, down regulation of gut granule biogenesis, down regulation of gut granule formation, down-regulation of gut granule assembly, down-regulation of gut granule biogenesis, down-regulation of gut granule formation, downregulation of gut granule assembly, downregulation of gut granule biogenesis, downregulation of gut granule formation, negative regulation of gut granule biogenesis, negative regulation of gut granule formation, inhibition of gut granule assembly, inhibition of gut granule biogenesis, inhibition of gut granule formation Relationships: is a type of negative regulation of organelle assembly [GO:1902116]; is a type of GO:1904755; negatively regulates gut granule assembly [GO:1902900] Definition: Any process that stops, prevents or reduces the frequency, rate or extent of gut granule assembly.